{
  "gene_symbol": "A0A8V8TLY5",
  "term_label": "Unknown biological process",
  "term_id": "UNKNOWN:0002",
  "gene": "UniProtKB:A0A8V8TLY5",
  "gene_name": "Ig-like domain-containing protein (Fragment)"
}